{
  "term_label": "Unknown molecular function",
  "gene_name": "RUN domain-containing protein 3B",
  "gene": "UniProtKB:Q96NL0",
  "gene_symbol": "RUNDC3B",
  "term_id": "UNKNOWN:0001"
}